protein heterooligomerization [GO:0051291] (BP) Also known as: protein heterooligomer assembly, protein heterooligomer biosynthesis, protein heterooligomer biosynthetic process, protein heterooligomer formation Relationships: is a type of protein complex oligomerization [GO:0051259] Sources: GOC:ai Subtypes: GO:0051290, protein heterotrimerization [GO:0070208] Definition: The process of creating protein oligomers, compounds composed of a small number, usually between three and ten, of component monomers that are not all identical. Oligomers may be formed by the polymerization of a number of monomers or the depolymerization of a large protein polymer.